{
  "gene_name": "Intraflagellar transport protein 27 homolog",
  "gene_symbol": "IFT27",
  "term_label": "Golgi membrane",
  "term_id": "GO:0000139",
  "gene": "UniProtKB:Q9BW83"
}